{
  "term_id": "GO:0031125",
  "gene_symbol": "REXO1",
  "term_label": "rRNA 3'-end processing",
  "gene_name": "RNA exonuclease 1 homolog",
  "gene": "UniProtKB:Q8N1G1"
}